{
  "gene_name": "Zinc finger protein 519",
  "gene": "UniProtKB:Q8TB69",
  "gene_symbol": "ZNF519",
  "term_label": "RNA polymerase II cis-regulatory region sequence-specific DNA binding",
  "term_id": "GO:0000978"
}